{
  "term_label": "Unknown molecular function",
  "gene": "UniProtKB:A1L1A6",
  "term_id": "UNKNOWN:0001",
  "gene_symbol": "IGSF23",
  "gene_name": "Immunoglobulin superfamily member 23"
}